{
  "gene": "UniProtKB:Q9GZW8",
  "gene_symbol": "MS4A7",
  "term_id": "GO:0005802",
  "gene_name": "Membrane-spanning 4-domains subfamily A member 7",
  "term_label": "trans-Golgi network"
}